metanephric glomerular mesangial cell proliferation involved in metanephros development [GO:0072262] (biological process) Definition: The multiplication or reproduction of glomerular mesangial cells in the metanephros, resulting in the expansion of the population. Subtypes: GO:0072263 Regulation: RO_0002211 by regulation of metanephric glomerular mesangial cell proliferation [GO:0072301]; negatively regulated by negative regulation of metanephric glomerular mesangial cell proliferation [GO:0072302]; positively regulated by GO:0072303 Sources: GOC:mtg_kidney_jan10 Relationships: is a type of GO:0072110; is a type of cell proliferation involved in metanephros development [GO:0072203]; is part of GO:0072223